{
  "gene": "UniProtKB:P0DMV8",
  "gene_name": "Heat shock 70 kDa protein 1A",
  "term_label": "cytosol",
  "term_id": "GO:0005829",
  "gene_symbol": "HSPA1A"
}